{
  "gene": "UniProtKB:Q14728",
  "gene_symbol": "MFSD10",
  "gene_name": "Major facilitator superfamily domain-containing protein 10",
  "term_id": "UNKNOWN:0002",
  "term_label": "Unknown biological process"
}